(carboxyethyl)arginine beta-lactam-synthase activity [GO:0034027] (molecular function) Relationships: is a type of GO:0016882 Sources: EC:6.3.3.4, RHEA:23620 Definition: Catalysis of the reaction: N(2)-(2-carboxyethyl)-L-arginine + ATP = AMP + deoxyamidinoproclavaminate + diphosphate + 2 H+. Also known as: L-2-N-(2-carboxyethyl)arginine cyclo-ligase (AMP-forming) activity, L-N2-(2-carboxyethyl)arginine cyclo-ligase (AMP-forming) activity, beta-lactam synthetase activity